{
  "gene_name": "ATPase GET3",
  "term_id": "GO:0043529",
  "gene_symbol": "GET3",
  "term_label": "GET complex",
  "gene": "UniProtKB:O43681"
}